{
  "gene": "UniProtKB:Q8TC99",
  "term_label": "Unknown molecular function",
  "gene_symbol": "FNDC8",
  "gene_name": "Fibronectin type III domain-containing protein 8",
  "term_id": "UNKNOWN:0001"
}